{
  "gene_symbol": "CHAC1",
  "term_id": "GO:0006751",
  "gene_name": "Glutathione-specific gamma-glutamylcyclotransferase 1",
  "term_label": "glutathione catabolic process",
  "gene": "UniProtKB:Q9BUX1"
}